{
  "term_label": "cytokine receptor activity",
  "gene_name": "Cytokine receptor common subunit beta",
  "gene": "UniProtKB:P32927",
  "term_id": "GO:0004896",
  "gene_symbol": "CSF2RB"
}